{
  "term_id": "GO:0031647",
  "gene_symbol": "USP47",
  "gene": "UniProtKB:Q96K76",
  "term_label": "regulation of protein stability",
  "gene_name": "Ubiquitin carboxyl-terminal hydrolase 47"
}